{
  "gene_name": "Glypican-5",
  "term_label": "cell surface",
  "gene": "UniProtKB:P78333",
  "gene_symbol": "GPC5",
  "term_id": "GO:0009986"
}